{
  "term_id": "GO:0005813",
  "gene_name": "Girdin",
  "gene_symbol": "CCDC88A",
  "term_label": "centrosome",
  "gene": "UniProtKB:Q3V6T2"
}